{
  "gene": "UniProtKB:Q2M2I5",
  "term_label": "keratin filament",
  "gene_symbol": "KRT24",
  "gene_name": "Keratin, type I cytoskeletal 24",
  "term_id": "GO:0045095"
}